{
  "gene_name": "Arf-GAP with GTPase, ANK repeat and PH domain-containing protein 11",
  "gene_symbol": "AGAP11",
  "term_id": "UNKNOWN:0003",
  "term_label": "Unknown cellular component",
  "gene": "UniProtKB:Q8TF27"
}